{
  "gene_symbol": "NDST1",
  "gene": "UniProtKB:P52848",
  "term_id": "GO:0015016",
  "gene_name": "Bifunctional heparan sulfate N-deacetylase_N-sulfotransferase 1",
  "term_label": "heparan sulfate N-sulfotransferase activity"
}